{
  "gene": "UniProtKB:O15254",
  "term_id": "GO:0005504",
  "term_label": "fatty acid binding",
  "gene_name": "Peroxisomal acyl-coenzyme A oxidase 3",
  "gene_symbol": "ACOX3"
}